{
  "term_label": "transcription coactivator activity",
  "gene_symbol": "JMY",
  "gene_name": "Junction-mediating and -regulatory protein",
  "gene": "UniProtKB:Q8N9B5",
  "term_id": "GO:0003713"
}